{
  "term_label": "regulation of ERK1 and ERK2 cascade",
  "term_id": "GO:0070372",
  "gene_symbol": "IL1A",
  "gene": "UniProtKB:P01583",
  "gene_name": "Interleukin-1 alpha"
}